clathrin-coated phagocytic vesicle [GO:0045336] (cellular component) Also known as: clathrin-coated phagosome Sources: GOC:go_curators, ISBN:0198506732 Relationships: is a type of clathrin-coated endocytic vesicle [GO:0045334]; is a type of phagocytic vesicle [GO:0045335] Definition: A clathrin-coated, membrane-bounded intracellular vesicle that arises from the ingestion of particulate material by phagocytosis.